{
  "term_label": "nucleus",
  "gene_symbol": "NRL",
  "gene": "UniProtKB:P54845",
  "term_id": "GO:0005634",
  "gene_name": "Neural retina-specific leucine zipper protein"
}